{
  "gene": "UniProtKB:Q14641",
  "gene_name": "Early placenta insulin-like peptide",
  "term_id": "UNKNOWN:0003",
  "gene_symbol": "INSL4",
  "term_label": "Unknown cellular component"
}